{
  "term_label": "Unknown biological process",
  "gene_symbol": "OR4F5",
  "term_id": "UNKNOWN:0002",
  "gene_name": "Olfactory receptor 4F5",
  "gene": "UniProtKB:Q8NH21"
}